{
  "gene": "UniProtKB:Q7Z2Z1",
  "term_label": "regulation of DNA-templated DNA replication initiation",
  "gene_name": "Treslin",
  "term_id": "GO:0030174",
  "gene_symbol": "TICRR"
}